{
  "gene_symbol": "SYCE2",
  "gene_name": "Synaptonemal complex central element protein 2",
  "term_label": "central element",
  "gene": "UniProtKB:Q6PIF2",
  "term_id": "GO:0000801"
}